{
  "gene_symbol": "GSDMA",
  "term_label": "pyroptotic inflammatory response",
  "gene_name": "Gasdermin-A",
  "gene": "UniProtKB:Q96QA5",
  "term_id": "GO:0070269"
}